positive regulation of invasive growth in response to glucose limitation [GO:2000219] (biological process) Relationships: is a type of positive regulation of growth of unicellular organism as a thread of attached cells [GO:0070786]; is a type of GO:2000217; positively regulates GO:0001403 Also known as: positive regulation of colony morphology Definition: Any process that activates or increases the frequency, rate or extent of invasive growth in response to glucose limitation. Sources: GOC:mah